{
  "gene_name": "Sodium_hydrogen exchanger 9B1",
  "gene": "UniProtKB:Q4ZJI4",
  "term_label": "Unknown cellular component",
  "gene_symbol": "SLC9B1",
  "term_id": "UNKNOWN:0003"
}